ferric enterobactin:proton symporter activity [GO:0015345] (molecular function) Also known as: ferric enterobactin:hydrogen symporter activity, ferric-enterobactin:proton symporter activity Definition: Enables the transfer of a solute or solutes from one side of a membrane to the other according to the reaction: ferric enterobactin(out) + H+(out) = ferric enterobactin(in) + H+(in). Sources: TC:2.A.1.16.2 Relationships: is a type of solute:proton symporter activity [GO:0015295]; is a type of iron chelate transmembrane transporter activity [GO:0015603]